{
  "term_id": "GO:0015721",
  "gene": "UniProtKB:G3V0H7",
  "term_label": "bile acid and bile salt transport",
  "gene_name": "Putative solute carrier organic anion transporter family member 1B7",
  "gene_symbol": "SLCO1B7"
}